{
  "gene": "UniProtKB:Q04743",
  "gene_symbol": "EMX2",
  "term_label": "DNA-binding transcription factor activity, RNA polymerase II-specific",
  "gene_name": "Homeobox protein EMX2",
  "term_id": "GO:0000981"
}